{
  "term_label": "ubiquitin-dependent protein catabolic process",
  "gene_name": "RING finger protein 215",
  "gene": "UniProtKB:Q9Y6U7",
  "gene_symbol": "RNF215",
  "term_id": "GO:0006511"
}